{
  "gene": "UniProtKB:Q9UN42",
  "term_id": "GO:0006355",
  "gene_symbol": "ATP1B4",
  "gene_name": "Protein ATP1B4",
  "term_label": "regulation of DNA-templated transcription"
}